{
  "gene_name": "DNA polymerase alpha subunit B",
  "gene": "UniProtKB:Q14181",
  "term_label": "alpha DNA polymerase:primase complex",
  "gene_symbol": "POLA2",
  "term_id": "GO:0005658"
}